spermine metabolic process [GO:0008215] (biological process) Sources: GOC:curators Definition: The chemical reactions and pathways involving spermine, a polybasic amine found in human sperm, in ribosomes and in some viruses, which is involved in nucleic acid packaging. Synthesis is regulated by ornithine decarboxylase which plays a key role in control of DNA replication. Relationships: is a type of polyamine metabolic process [GO:0006595] Subtypes: spermine biosynthetic process [GO:0006597], arginine catabolic process to spermine [GO:0019548], GO:0032919, spermine catabolic process [GO:0046208] Also known as: spermine metabolism